{
  "gene_name": "Zinc finger protein 772",
  "term_id": "GO:0005634",
  "gene": "UniProtKB:Q68DY9",
  "gene_symbol": "ZNF772",
  "term_label": "nucleus"
}